{
  "gene_name": "Claudin-2",
  "gene": "UniProtKB:P57739",
  "term_id": "GO:0160184",
  "gene_symbol": "CLDN2",
  "term_label": "paracellular transport"
}